{
  "term_label": "nucleoplasm",
  "gene_name": "Zinc finger and BTB domain-containing protein 39",
  "gene_symbol": "ZBTB39",
  "gene": "UniProtKB:O15060",
  "term_id": "GO:0005654"
}